{
  "gene": "UniProtKB:Q15493",
  "gene_symbol": "RGN",
  "term_label": "L-ascorbic acid biosynthetic process",
  "term_id": "GO:0019853",
  "gene_name": "Regucalcin"
}